{
  "term_id": "GO:0005829",
  "gene_symbol": "TIAM1",
  "term_label": "cytosol",
  "gene": "UniProtKB:Q13009",
  "gene_name": "Rho guanine nucleotide exchange factor TIAM1"
}